{
  "gene": "UniProtKB:P42229",
  "gene_name": "Signal transducer and activator of transcription 5A",
  "term_id": "GO:0006357",
  "gene_symbol": "STAT5A",
  "term_label": "regulation of transcription by RNA polymerase II"
}